{
  "gene_name": "Mas-related G-protein coupled receptor member X2",
  "term_label": "G protein-coupled receptor activity",
  "gene_symbol": "MRGPRX2",
  "term_id": "GO:0004930",
  "gene": "UniProtKB:Q96LB1"
}